peptide catabolic process [GO:0043171] (biological process) Sources: GOC:jl Relationships: is a type of peptide metabolic process [GO:0006518]; is_a catabolic process [GO:0009056] Also known as: peptide breakdown, peptide catabolism, peptide degradation Subtypes: GO:0010813, peptide antibiotic catabolic process [GO:0030652] Definition: The chemical reactions and pathways resulting in the breakdown of peptides, compounds of 2 or more (but usually less than 100) amino acids where the alpha carboxyl group of one is bound to the alpha amino group of another.